{
  "gene": "UniProtKB:Q86UL8",
  "gene_name": "Membrane-associated guanylate kinase, WW and PDZ domain-containing protein 2",
  "term_label": "cell-cell junction",
  "gene_symbol": "MAGI2",
  "term_id": "GO:0005911"
}